{
  "term_label": "ubiquitin binding",
  "gene": "UniProtKB:Q96FW1",
  "gene_name": "Ubiquitin thioesterase OTUB1",
  "gene_symbol": "OTUB1",
  "term_id": "GO:0043130"
}